{
  "gene_symbol": "CNTF",
  "term_id": "GO:0007259",
  "gene_name": "Ciliary neurotrophic factor",
  "term_label": "cell surface receptor signaling pathway via JAK-STAT",
  "gene": "UniProtKB:P26441"
}